neutral amino acid, sodium:proton antiporter activity [GO:0140893] (molecular function) Definition: Enables the transfer of a solute or solutes from one side of a membrane to the other according to the reaction: H+(in) + amino acid(out) + Na+(out) = H+(out) + amino acid(in) + Na+(in). References: PMID:11698233, PMID:34704597 Also known as: amino acid-coupled Na+/H+ exchanger activity Relationships: is a type of sodium:proton antiporter activity [GO:0015385]